{
  "gene_symbol": "FAAH2",
  "term_id": "UNKNOWN:0001",
  "gene": "UniProtKB:Q6GMR7",
  "gene_name": "Fatty-acid amide hydrolase 2",
  "term_label": "Unknown molecular function"
}